{
  "term_label": "structural constituent of ribosome",
  "gene_name": "Large ribosomal subunit protein eL21",
  "term_id": "GO:0003735",
  "gene": "UniProtKB:P46778",
  "gene_symbol": "RPL21"
}